axolemma [GO:0030673] (cellular component) Also known as: axonal membrane Definition: The portion of the plasma membrane surrounding an axon; it is a specialized trilaminar random mosaic of protein molecules floating within a fluid matrix of highly mobile phospholipid molecules, 7-8 nm in thickness. Relationships: is a type of neuron projection membrane [GO:0032589]; is part of main axon [GO:0044304] References: PMID:9527135